{
  "gene_symbol": "NDUFAF8",
  "gene": "UniProtKB:A1L188",
  "gene_name": "NADH dehydrogenase [ubiquinone] 1 alpha subcomplex assembly factor 8",
  "term_label": "mitochondrial respiratory chain complex I assembly",
  "term_id": "GO:0032981"
}